L-methylmalonyl-CoA metabolic process [GO:0046491] (biological process) Subtypes: L-methylmalonyl-CoA biosynthetic process [GO:0019680] Also known as: L-methylmalonyl-CoA metabolism Sources: GOC:jsg, GOC:mah, ISBN:0198506732 Definition: The chemical reactions and pathways involving L-methylmalonyl-CoA, the L-enantiomer of 2-carboxypropanoyl-CoA. S-methylmalonyl-CoA is an intermediate in the beta oxidation of odd-numbered fatty acids in animals. Relationships: is_a acyl-CoA metabolic process [GO:0006637]